{
  "term_id": "GO:0006744",
  "term_label": "ubiquinone biosynthetic process",
  "gene_symbol": "COQ8A",
  "gene_name": "Atypical kinase COQ8A, mitochondrial",
  "gene": "UniProtKB:Q8NI60"
}